{
  "gene_symbol": "PPP1R9B",
  "term_label": "postsynaptic density",
  "gene": "UniProtKB:Q96SB3",
  "gene_name": "Neurabin-2",
  "term_id": "GO:0014069"
}